{
  "term_label": "Unknown biological process",
  "gene_name": "Small integral membrane protein 39",
  "gene_symbol": "SMIM39",
  "term_id": "UNKNOWN:0002",
  "gene": "UniProtKB:A0A1B0GW54"
}